N-acylmannosamine kinase activity [GO:0009384] (molecular function) Sources: EC:2.7.1.60 Definition: Catalysis of the reaction: ATP + N-acyl-D-mannosamine = ADP + N-acyl-D-mannosamine 6-phosphate. Also known as: ATP:N-acetylmannosamine 6-phosphotransferase activity, ATP:N-acyl-D-mannosamine 6-phosphotransferase activity, N-acetylmannosamine kinase activity, N-acyl-D-mannosamine kinase activity, acetylamidodeoxymannokinase activity, acetylmannosamine kinase activity, acylaminodeoxymannokinase activity, acylmannosamine kinase (phosphorylating), acylmannosamine kinase activity Relationships: is a type of GO:0016773; is a type of GO:0019200